furylfuramide isomerase activity [GO:0047907] (molecular function) Also known as: 2-(2-furyl)-3-(5-nitro-2-furyl)acrylamide cis-trans-isomerase activity Sources: EC:5.2.1.6, RHEA:21848 Definition: Catalysis of the reaction: (E)-2-(2-furyl)-3-(5-nitro-2-furyl)acrylamide = (Z)-2-(2-furyl)-3-(5-nitro-2-furyl)acrylamide. Relationships: is a type of cis-trans isomerase activity [GO:0016859]